G protein-coupled photoreceptor activity [GO:0008020] (molecular function) Sources: GOC:bf, GOC:dph, ISBN:0198506732 Definition: Combining with incidental electromagnetic radiation, particularly visible light, and transmitting the signal across the membrane by activating an associated G-protein; promotes the exchange of GDP for GTP on the alpha subunit of a heterotrimeric G-protein complex. Relationships: is a type of G protein-coupled receptor activity [GO:0004930]; is a type of photoreceptor activity [GO:0009881]; is part of detection of visible light [GO:0009584] Also known as: G protein coupled photoreceptor activity, G-protein coupled photoreceptor activity, photoreceptor activity, G-protein coupled